{
  "gene_name": "Tubulin-specific chaperone cofactor E-like protein",
  "gene": "UniProtKB:Q5QJ74",
  "gene_symbol": "TBCEL",
  "term_id": "GO:0000226",
  "term_label": "microtubule cytoskeleton organization"
}